{
  "term_label": "regulation of transcription by RNA polymerase II",
  "gene": "UniProtKB:Q9H9D4",
  "gene_name": "Zinc finger protein 408",
  "term_id": "GO:0006357",
  "gene_symbol": "ZNF408"
}